{
  "gene": "UniProtKB:Q86UU0",
  "term_label": "beta-catenin-TCF complex",
  "gene_name": "B-cell CLL_lymphoma 9-like protein",
  "term_id": "GO:1990907",
  "gene_symbol": "BCL9L"
}